{
  "gene_symbol": "DRAP1",
  "gene_name": "Dr1-associated corepressor",
  "term_id": "GO:0001046",
  "gene": "UniProtKB:Q14919",
  "term_label": "core promoter sequence-specific DNA binding"
}